{
  "gene_symbol": "PVRIG",
  "term_id": "GO:0005886",
  "gene": "UniProtKB:Q6DKI7",
  "term_label": "plasma membrane",
  "gene_name": "Transmembrane protein PVRIG"
}